{
  "gene_name": "Nucleosome-remodeling factor subunit BPTF",
  "gene": "UniProtKB:Q12830",
  "gene_symbol": "BPTF",
  "term_id": "GO:0006357",
  "term_label": "regulation of transcription by RNA polymerase II"
}